{
  "term_id": "UNKNOWN:0002",
  "gene_symbol": "ANKRD19P",
  "gene": "UniProtKB:Q9H560",
  "term_label": "Unknown biological process",
  "gene_name": "Putative ankyrin repeat domain-containing protein 19"
}